{
  "gene_symbol": "DHTKD1",
  "term_id": "UNKNOWN:0003",
  "gene_name": "2-oxoadipate dehydrogenase complex component E1",
  "gene": "UniProtKB:Q96HY7",
  "term_label": "Unknown cellular component"
}